peripheral B cell deletion [GO:0002454] (biological process) Definition: The deletion of B cells by apoptotic process occurring as part of peripheral tolerance induction and B cell selection. Also known as: peripheral B lymphocyte deletion, peripheral B-cell deletion, peripheral B-lymphocyte deletion Relationships: is a type of GO:0002516; BFO_0000050 peripheral B cell tolerance induction [GO:0002451] Sources: GOC:add, GOC:jal, GOC:mtg_apoptosis, ISBN:0781735149 Regulation: regulated by regulation of peripheral B cell deletion [GO:0002908]; negatively regulated by negative regulation of peripheral B cell deletion [GO:0002909]; positively regulated by GO:0002910